{
  "gene_symbol": "APH1A",
  "term_label": "amyloid-beta formation",
  "gene_name": "Gamma-secretase subunit APH-1A",
  "term_id": "GO:0034205",
  "gene": "UniProtKB:Q96BI3"
}